{
  "term_label": "Unknown biological process",
  "gene_symbol": "SDR42E1",
  "term_id": "UNKNOWN:0002",
  "gene": "UniProtKB:Q8WUS8",
  "gene_name": "Short-chain dehydrogenase_reductase family 42E member 1"
}